{
  "gene": "UniProtKB:Q75QN2",
  "term_id": "GO:0032039",
  "gene_name": "Integrator complex subunit 8",
  "term_label": "integrator complex",
  "gene_symbol": "INTS8"
}